{
  "gene": "UniProtKB:Q8WVM8",
  "gene_symbol": "SCFD1",
  "term_label": "intracellular protein transport",
  "gene_name": "Sec1 family domain-containing protein 1",
  "term_id": "GO:0006886"
}